D-galacturonate catabolic process [GO:0019698] (BP) Definition: The chemical reactions and pathways resulting in the breakdown of D-galacturonate, the D-enantiomer of galacturonate, the anion of galacturonic acid. Sources: GOC:ai, GOC:jsg, GOC:mah Also known as: D-galacturonate breakdown, D-galacturonate catabolism, D-galacturonate degradation Relationships: is a type of monosaccharide catabolic process [GO:0046365]; is a type of GO:0046396; is a type of galacturonate catabolic process [GO:0046397]